mitotic checkpoint complex [GO:0033597] (cellular component) References: PMID:10704439, PMID:11535616, PMID:11726501, PMID:17650307 Also known as: MCC Definition: A multiprotein complex that functions as a mitotic checkpoint inhibitor of the anaphase-promoting complex/cyclosome (APC/C). In budding yeast this complex consists of Mad2p, Mad3p, Bub3p and Cdc20p, and in mammalian cells it consists of MAD2, BUBR1, BUB3, and CDC20. Relationships: is a type of nuclear protein-containing complex [GO:0140513]; has part GO:1990298